(S)-2-hydroxyglutarate dehydrogenase activity [GO:0047545] (molecular function) Definition: Catalysis of the reaction: (S)-2-hydroxyglutarate + acceptor = 2-oxoglutarate + reduced acceptor. Sources: RHEA:21252 Also known as: 2-hydroxyglutarate dehydrogenase activity, L-alpha-hydroxyglutarate:NAD+ 2-oxidoreductase, alpha-hydroxyglutarate dehydrogenase (NAD+ specific), (S)-2-hydroxyglutarate:(acceptor) 2-oxidoreductase, (S)-2-hydroxyglutarate:acceptor 2-oxidoreductase, L-alpha-hydroxyglutarate dehydrogenase activity, alpha-hydroxyglutarate dehydrogenase activity, alpha-hydroxyglutarate oxidoreductase activity, hydroxyglutaric dehydrogenase activity Relationships: is a type of GO:0016614 Subtypes: (S)-2-hydroxyglutarate dehydrogenase (quinone) activity [GO:0140696]